histone H3R17 methyltransferase activity [GO:0035642] (molecular function) Also known as: histone methylase activity (H3-R17 specific), histone methyltransferase activity (H3-R17 specific), histone-H3R17 methyltransferase activity, histone-arginine N-methyltransferase activity (H3-R17 specific) Relationships: is a type of protein-arginine N-methyltransferase activity [GO:0016274]; is a type of histone H3 methyltransferase activity [GO:0140938] References: PMID:11341840 Note: Comment: Note that the residue position corresponds to the canonical human H3 histone (UniProtKB:P84243); this residue is conserved across all eukaryotes. Residue 1 is the first residue following removal of the initiating Methionine (Met). Note that each histone is encoded by multiple genes, and sequences may vary across different genes within an organism. Definition: Catalysis of the reaction: S-adenosyl-L-methionine + (histone H3)-arginine (position 17) = S-adenosyl-L-homocysteine + (histone H3)-N-methyl-arginine (position 17). This reaction is the addition of a methyl group to the arginine residue at position 17 of histone H3.